{
  "term_label": "protein-membrane adaptor activity",
  "gene": "UniProtKB:Q8N3P4",
  "gene_name": "Vacuolar protein sorting-associated protein 8 homolog",
  "term_id": "GO:0043495",
  "gene_symbol": "VPS8"
}